{
  "gene_symbol": "OTX2",
  "gene": "UniProtKB:P32243",
  "term_label": "RNA polymerase II cis-regulatory region sequence-specific DNA binding",
  "gene_name": "Homeobox protein OTX2",
  "term_id": "GO:0000978"
}